{
  "gene_symbol": "SPIRE1",
  "term_label": "polar body extrusion after meiotic divisions",
  "gene_name": "Protein spire homolog 1",
  "term_id": "GO:0040038",
  "gene": "UniProtKB:Q08AE8"
}